{
  "term_label": "Unknown molecular function",
  "gene_symbol": "GPR68",
  "term_id": "UNKNOWN:0001",
  "gene": "UniProtKB:Q15743",
  "gene_name": "Ovarian cancer G-protein coupled receptor 1"
}